{
  "term_id": "GO:0030154",
  "term_label": "cell differentiation",
  "gene_name": "Proto-oncogene tyrosine-protein kinase Src",
  "gene_symbol": "SRC",
  "gene": "UniProtKB:P12931"
}